positive regulation of kidney smooth muscle cell differentiation [GO:2000358] (biological process) Relationships: is a type of positive regulation of smooth muscle cell differentiation [GO:0051152]; is a type of GO:2000356; positively regulates GO:0072195 Definition: Any process that activates or increases the frequency, rate or extent of kidney smooth muscle cell differentiation. Sources: GOC:obol